{
  "gene_symbol": "AKR1C4",
  "gene_name": "Aldo-keto reductase family 1 member C4",
  "term_id": "GO:0044598",
  "gene": "UniProtKB:P17516",
  "term_label": "doxorubicin metabolic process"
}